{
  "term_label": "phosphatidylinositol phosphate biosynthetic process",
  "term_id": "GO:0046854",
  "gene": "UniProtKB:P42356",
  "gene_name": "Phosphatidylinositol 4-kinase alpha",
  "gene_symbol": "PI4KA"
}